posterior midgut invagination [GO:0007374] (biological process) Relationships: is a type of embryonic morphogenesis [GO:0048598]; is a type of morphogenesis of an epithelial fold [GO:0060571]; BFO_0000050 gastrulation involving germ band extension [GO:0010004] Sources: ISBN:0879694238 Definition: Formation of a cup-shaped invagination at the posterior end of the embryo, bringing the posterior midgut and hindgut primordia into the interior.